negative regulation of cardiac muscle tissue regeneration [GO:1905179] (biological process) References: PMID:23222520 Sources: GOC:BHF, GOC:BHF_miRNA, GOC:TermGenie, GOC:rph, GO_REF:0000058 Also known as: down regulation of cardiac muscle tissue regeneration, down-regulation of cardiac muscle tissue regeneration, downregulation of cardiac muscle tissue regeneration, inhibition of cardiac muscle tissue regeneration Relationships: is_a negative regulation of developmental growth [GO:0048640]; is a type of regulation of cardiac muscle tissue regeneration [GO:1905178]; negatively regulates cardiac muscle tissue regeneration [GO:0061026] Definition: Any process that stops, prevents or reduces the frequency, rate or extent of cardiac muscle tissue regeneration.